adult locomotory behavior [GO:0008344] (biological process) Subtypes: adult walking behavior [GO:0007628], flight behavior [GO:0007629], jump response [GO:0007630] Relationships: is a type of GO:0007626; is_a adult behavior [GO:0030534] Sources: GOC:ai Note: See also the biological process term 'locomotory behavior ; GO:0007626'. Also known as: adult locomotory behaviour Definition: Locomotory behavior in a fully developed and mature organism.